{
  "term_id": "GO:0042613",
  "gene": "UniProtKB:P06340",
  "term_label": "MHC class II protein complex",
  "gene_symbol": "HLA-DOA",
  "gene_name": "HLA class II histocompatibility antigen, DO alpha chain"
}